{
  "gene_name": "Centrosome-associated protein ALMS1",
  "gene": "UniProtKB:Q8TCU4",
  "term_id": "GO:0005829",
  "term_label": "cytosol",
  "gene_symbol": "ALMS1"
}